{
  "gene_name": "Myozenin-2",
  "gene": "UniProtKB:Q9NPC6",
  "term_id": "GO:0030018",
  "gene_symbol": "MYOZ2",
  "term_label": "Z disc"
}